{
  "gene": "UniProtKB:P15976",
  "term_label": "negative regulation of transcription by RNA polymerase II",
  "term_id": "GO:0000122",
  "gene_name": "Erythroid transcription factor",
  "gene_symbol": "GATA1"
}